{
  "term_id": "GO:0005737",
  "gene_symbol": "KIF20A",
  "term_label": "cytoplasm",
  "gene_name": "Kinesin-like protein KIF20A",
  "gene": "UniProtKB:O95235"
}